{
  "gene_name": "Golgi-associated plant pathogenesis-related protein 1",
  "term_label": "Unknown molecular function",
  "term_id": "UNKNOWN:0001",
  "gene": "UniProtKB:Q9H4G4",
  "gene_symbol": "GLIPR2"
}